{
  "gene": "UniProtKB:Q9Y2E6",
  "term_label": "Notch signaling pathway",
  "gene_name": "E3 ubiquitin-protein ligase DTX4",
  "term_id": "GO:0007219",
  "gene_symbol": "DTX4"
}